{
  "gene_symbol": "PHYHD1",
  "term_label": "Unknown cellular component",
  "gene_name": "Phytanoyl-CoA dioxygenase domain-containing protein 1",
  "gene": "UniProtKB:Q5SRE7",
  "term_id": "UNKNOWN:0003"
}